{
  "gene_name": "Platelet glycoprotein 4",
  "term_label": "scavenger receptor activity",
  "gene": "UniProtKB:P16671",
  "gene_symbol": "CD36",
  "term_id": "GO:0005044"
}